regulation of cytokine production involved in inflammatory response [GO:1900015] (biological process) Relationships: is a type of regulation of cytokine production [GO:0001817]; regulates cytokine production involved in inflammatory response [GO:0002534] Subtypes: GO:1900016, GO:1900017 Also known as: regulation of cytokine production involved in acute inflammatory response Sources: GOC:TermGenie Definition: Any process that modulates the frequency, rate or extent of cytokine production involved in inflammatory response.